{
  "term_label": "Unknown cellular component",
  "gene": "UniProtKB:Q96TA1",
  "gene_symbol": "NIBAN2",
  "term_id": "UNKNOWN:0003",
  "gene_name": "Protein Niban 2"
}